{
  "gene_symbol": "RGPD8",
  "gene": "UniProtKB:O14715",
  "gene_name": "RANBP2-like and GRIP domain-containing protein 8",
  "term_label": "SUMO transferase activity",
  "term_id": "GO:0019789"
}